ganglion structural organization [GO:0061555] (biological process) Subtypes: GO:0061562 Definition: The process that contributes to creating the structural organization of a ganglion. This process pertains to the physical shaping of a rudimentary structure. Also known as: ganglia structural organization Relationships: is a type of anatomical structure arrangement [GO:0048532]; is part of GO:0061552 Sources: GOC:dph